{
  "term_id": "GO:0030141",
  "gene_name": "Kallikrein-11",
  "gene_symbol": "KLK11",
  "gene": "UniProtKB:Q9UBX7",
  "term_label": "secretory granule"
}